positive regulation of cellular response to alcohol [GO:1905959] (biological process) Relationships: is a type of positive regulation of cellular process [GO:0048522]; is a type of GO:1901421; is a type of regulation of cellular response to alcohol [GO:1905957]; positively regulates GO:0097306 Definition: Any process that activates or increases the frequency, rate or extent of cellular response to alcohol. References: PMID:26434723 Sources: GOC:TermGenie, GO_REF:0000058 Also known as: up regulation of cellular response to alcohol, up-regulation of cellular response to alcohol, upregulation of cellular response to alcohol, activation of cellular response to alcohol